{
  "gene_symbol": "SEPTIN4",
  "term_id": "GO:0060090",
  "term_label": "molecular adaptor activity",
  "gene_name": "Septin-4",
  "gene": "UniProtKB:O43236"
}